{
  "gene_name": "BDNF_NT-3 growth factors receptor",
  "gene": "UniProtKB:Q16620",
  "term_id": "GO:0014069",
  "gene_symbol": "NTRK2",
  "term_label": "postsynaptic density"
}